{
  "gene": "UniProtKB:P35346",
  "term_label": "neuropeptide signaling pathway",
  "gene_name": "Somatostatin receptor type 5",
  "term_id": "GO:0007218",
  "gene_symbol": "SSTR5"
}